{
  "term_id": "GO:0071546",
  "gene_name": "Ankyrin repeat domain-containing protein 34B",
  "gene": "UniProtKB:A5PLL1",
  "gene_symbol": "ANKRD34B",
  "term_label": "pi-body"
}